{
  "gene_name": "Protein FAM240A",
  "gene": "UniProtKB:A0A1B0GVK7",
  "gene_symbol": "FAM240A",
  "term_id": "UNKNOWN:0001",
  "term_label": "Unknown molecular function"
}